arabinose transmembrane transporter activity [GO:0042900] (molecular function) Relationships: is a type of pentose transmembrane transporter activity [GO:0015146]; is part of GO:0015751 Definition: Enables the transfer of arabinose, a pentose monosaccharide that occurs in both D and L configurations, and as a polymer, from one side of a membrane to the other. Subtypes: GO:0015147, GO:0015518 Sources: GOC:jl, GOC:mtg_transport, ISBN:0815340729